{
  "term_label": "aspartic-type endopeptidase activity",
  "gene": "UniProtKB:Q9Y5Z0",
  "gene_name": "Beta-secretase 2",
  "gene_symbol": "BACE2",
  "term_id": "GO:0004190"
}